regulation of purine nucleobase metabolic process [GO:0006141] (biological process) Sources: GOC:go_curators Also known as: regulation of purine base metabolic process, regulation of purine base metabolism Subtypes: negative regulation of purine nucleobase metabolic process [GO:0045982], positive regulation of purine nucleobase metabolic process [GO:0045983], regulation of adenine biosynthetic process [GO:0061934] Definition: Any process that modulates the frequency, rate or extent of the chemical reactions and pathways involving purines. Relationships: is a type of regulation of nucleobase-containing compound metabolic process [GO:0019219]; is a type of regulation of small molecule metabolic process [GO:0062012]; regulates GO:0006144